{
  "term_label": "Unknown biological process",
  "term_id": "UNKNOWN:0002",
  "gene_symbol": "C16orf78",
  "gene": "UniProtKB:Q8WTQ4",
  "gene_name": "Uncharacterized protein C16orf78"
}